galactose 3-O-sulfotransferase activity [GO:0050694] (molecular function) Relationships: is a type of sulfotransferase activity [GO:0008146] Subtypes: galactosylceramide sulfotransferase activity [GO:0001733] Definition: Catalysis of the reaction: N-acetyllactosamine + 3'-phosphoadenosine 5'-phosphosulfate = 3-sulfo-N-acetyllactosamine + adenosine 3',5'-bisphosphate. N-acetyllactosamine residues are found in a number of different carbohydrate types. N-acetyllactosamine can also be written as Gal-beta-(1,4)-GlcNAc. References: PMID:11323440, PMID:11356829 Sources: GOC:ai Also known as: Gal-3-O-sulfotransferase activity, galactose 3-O-sulphotransferase activity